{
  "gene": "UniProtKB:P24386",
  "gene_name": "Rab proteins geranylgeranyltransferase component A 1",
  "term_label": "vesicle-mediated transport",
  "gene_symbol": "CHM",
  "term_id": "GO:0016192"
}